positive regulation of filamentous growth [GO:0090033] (biological process) Subtypes: positive regulation of filamentous growth of a population of unicellular organisms [GO:1900430] Definition: Any process that increases the frequency, rate or extent of the process in which a multicellular organism or a group of unicellular organisms grow in a threadlike, filamentous shape. Relationships: is a type of regulation of filamentous growth [GO:0010570]; is a type of positive regulation of growth [GO:0045927]; positively regulates filamentous growth [GO:0030447] Sources: GOC:dph, GOC:tb